single-species biofilm formation [GO:0044010] (biological process) Definition: A process in which planktonically growing microorganisms of the same species grow at a liquid-air interface or on a solid substrate under the flow of a liquid and produce extracellular polymers that facilitate matrix formation, resulting in a change in the organisms' growth rate and gene transcription. Sources: GOC:cc, GOC:di, GOC:tb Also known as: auto-aggregation, bfp-dependent aggregation, bundle-forming fimbriae-dependent aggregation, bundle-forming pili-dependent aggregation, tfp-dependent aggregation, type IV pili-dependent aggregation Relationships: is a type of biofilm formation [GO:0042710]; is a type of GO:0051703 Subtypes: single-species biofilm formation in or on host organism [GO:0044407], single-species surface biofilm formation [GO:0090606], GO:0090609 Regulation: regulated by GO:1900190; negatively regulated by GO:1900191; positively regulated by positive regulation of single-species biofilm formation [GO:1900192]